{
  "gene_symbol": "PICK1",
  "gene_name": "PRKCA-binding protein",
  "term_id": "GO:0005543",
  "gene": "UniProtKB:Q9NRD5",
  "term_label": "phospholipid binding"
}